{
  "gene": "UniProtKB:Q9Y3R4",
  "term_id": "GO:0016020",
  "gene_name": "Sialidase-2",
  "term_label": "membrane",
  "gene_symbol": "NEU2"
}